nuclear retinoic acid receptor binding [GO:0042974] (molecular function) References: PMID:12476796 Sources: GOC:jl Also known as: retinoic acid receptor binding, RAR binding Relationships: is a type of nuclear receptor binding [GO:0016922] Definition: Binding to a nuclear retinoic acid receptor, a ligand-regulated transcription factor belonging to the nuclear receptor superfamily. Subtypes: GO:0046965